positive regulation of fever generation [GO:0031622] (BP) Subtypes: positive regulation of fever generation by positive regulation of prostaglandin biosynthesis [GO:0071811], positive regulation of fever generation by positive regulation of prostaglandin secretion [GO:0071812] Sources: GOC:add Definition: Any process that activates or increases the frequency, rate, or extent of fever generation. Also known as: positive regulation of pyrexia, up regulation of fever, up-regulation of fever, upregulation of fever, activation of fever, stimulation of fever Relationships: is a type of GO:0002675; is_a regulation of fever generation [GO:0031620]; is_a positive regulation of heat generation [GO:0031652]; positively regulates fever generation [GO:0001660]